{
  "gene": "UniProtKB:O14842",
  "term_id": "GO:0007204",
  "gene_symbol": "FFAR1",
  "gene_name": "Free fatty acid receptor 1",
  "term_label": "positive regulation of cytosolic calcium ion concentration"
}